{
  "term_id": "GO:0005930",
  "term_label": "axoneme",
  "gene": "UniProtKB:Q9UHG0",
  "gene_symbol": "DCDC2",
  "gene_name": "Doublecortin domain-containing protein 2"
}